{
  "gene_name": "Uncharacterized protein FLJ30774",
  "term_id": "UNKNOWN:0002",
  "gene": "UniProtKB:Q96NJ1",
  "term_label": "Unknown biological process",
  "gene_symbol": "Q96NJ1"
}